{
  "gene_symbol": "GSK3B",
  "term_id": "GO:0010508",
  "gene": "UniProtKB:P49841",
  "term_label": "positive regulation of autophagy",
  "gene_name": "Glycogen synthase kinase-3 beta"
}